{
  "gene_name": "Telomerase Cajal body protein 1",
  "gene_symbol": "WRAP53",
  "term_label": "RNA binding",
  "term_id": "GO:0003723",
  "gene": "UniProtKB:Q9BUR4"
}